{
  "gene": "UniProtKB:Q6DD88",
  "term_label": "endoplasmic reticulum organization",
  "gene_symbol": "ATL3",
  "term_id": "GO:0007029",
  "gene_name": "Atlastin-3"
}